{
  "gene_name": "Chorionic somatomammotropin hormone-like 1",
  "term_id": "GO:0060396",
  "term_label": "growth hormone receptor signaling pathway",
  "gene_symbol": "CSHL1",
  "gene": "UniProtKB:Q14406"
}